{
  "gene_name": "Myeloperoxidase",
  "gene": "UniProtKB:P05164",
  "term_id": "GO:0004601",
  "term_label": "peroxidase activity",
  "gene_symbol": "MPO"
}